cyclopentanol catabolic process [GO:0033022] (biological process) Relationships: is a type of alcohol catabolic process [GO:0046164] References: PMID:12406764 Sources: GOC:mah Also known as: cyclopentanol breakdown, cyclopentanol catabolism, cyclopentanol degradation Definition: The chemical reactions and pathways resulting in the breakdown of cyclopentanol.